{
  "gene_name": "Immunoglobulin kappa variable 5-2",
  "gene_symbol": "IGKV5-2",
  "gene": "UniProtKB:P06315",
  "term_label": "immunoglobulin complex",
  "term_id": "GO:0019814"
}